{
  "gene": "UniProtKB:P46597",
  "gene_name": "Acetylserotonin O-methyltransferase",
  "term_label": "melatonin biosynthetic process",
  "term_id": "GO:0030187",
  "gene_symbol": "ASMT"
}